{
  "gene_name": "Protein JTB",
  "term_label": "spindle",
  "gene_symbol": "JTB",
  "gene": "UniProtKB:O76095",
  "term_id": "GO:0005819"
}